profilin binding [GO:0005522] (molecular function) Definition: Binding to profilin, an actin-binding protein that forms a complex with G-actin and prevents it from polymerizing to form F-actin. Sources: ISBN:0721662544 Relationships: is a type of GO:0005515